{
  "gene": "UniProtKB:P49758",
  "gene_name": "Regulator of G-protein signaling 6",
  "term_id": "GO:0007186",
  "gene_symbol": "RGS6",
  "term_label": "G protein-coupled receptor signaling pathway"
}